{
  "gene_symbol": "TIPIN",
  "term_label": "replication fork protection complex",
  "term_id": "GO:0031298",
  "gene": "UniProtKB:Q9BVW5",
  "gene_name": "TIMELESS-interacting protein"
}